{
  "gene_name": "AN1-type zinc finger protein 2A",
  "term_id": "GO:0043161",
  "gene_symbol": "ZFAND2A",
  "gene": "UniProtKB:Q8N6M9",
  "term_label": "proteasome-mediated ubiquitin-dependent protein catabolic process"
}